positive extrathymic T cell selection [GO:0045067] (biological process) Also known as: positive extrathymic T lymphocyte selection, positive extrathymic T-cell selection, positive extrathymic T-lymphocyte selection References: PMID:7880383 Sources: ISBN:0781735149 Definition: The process of sparing extrathymically maturing T cells which react with self-MHC protein complexes with low affinity levels from apoptotic death. Relationships: is a type of GO:0043368; is a type of GO:0045062